labyrinthine layer development [GO:0060711] (biological process) Sources: GOC:dph Definition: The process in which the labyrinthine layer of the placenta progresses, from its formation to its mature state. Relationships: is_a GO:0048856; is part of embryonic placenta development [GO:0001892]